membrane repolarization during cardiac muscle cell action potential [GO:0086013] (BP) Subtypes: GO:0086049, GO:0086050, membrane repolarization during Purkinje myocyte action potential [GO:0086051], membrane repolarization during SA node cell action potential [GO:0086052], GO:0098914, membrane repolarization during ventricular cardiac muscle cell action potential [GO:0098915] Regulation: regulated by regulation of membrane repolarization during cardiac muscle cell action potential [GO:1905031]; negatively regulated by GO:1905032; positively regulated by positive regulation of membrane repolarization during cardiac muscle cell action potential [GO:1905033] Definition: The process in which ions are transported across a membrane such that the cardiac muscle cell plasma membrane potential changes in the direction from the positive membrane potential at the peak of the action potential towards the negative resting potential. Sources: GOC:BHF, GOC:mtg_cardiac_conduct_nov11 Relationships: is a type of membrane repolarization during action potential [GO:0086011]; is a type of cardiac muscle cell membrane repolarization [GO:0099622]; is part of cardiac muscle cell action potential [GO:0086001]